{
  "term_label": "endoplasmic reticulum to Golgi vesicle-mediated transport",
  "gene": "UniProtKB:Q5JRA6",
  "gene_symbol": "MIA3",
  "gene_name": "Transport and Golgi organization protein 1 homolog",
  "term_id": "GO:0006888"
}